noradrenergic neuron fate commitment [GO:0003359] (biological process) Sources: GOC:dph Relationships: is a type of GO:0048663; is part of noradrenergic neuron differentiation [GO:0003357] Definition: The process in which the developmental fate of a cell becomes restricted such that it will develop into a noradrenergic neuron. Subtypes: noradrenergic neuron fate commitment involved in brainstem development [GO:0003362] Also known as: norepinephrine secreting neuron fate commitment